{
  "gene_symbol": "BUB1",
  "gene_name": "Mitotic checkpoint serine_threonine-protein kinase BUB1",
  "gene": "UniProtKB:O43683",
  "term_id": "GO:0000776",
  "term_label": "kinetochore"
}